plasma membrane ATP synthesis coupled electron transport [GO:0042774] (biological process) Definition: The transfer of electrons through a series of electron donors and acceptors, generating energy that is ultimately used for synthesis of ATP in the plasma membrane. Sources: GOC:mtg_sensu, ISBN:0716731363 Relationships: is a type of GO:0042773; occurs in plasma membrane [GO:0005886]